{
  "gene": "UniProtKB:Q9P2D3",
  "gene_symbol": "HEATR5B",
  "term_id": "GO:0030139",
  "gene_name": "HEAT repeat-containing protein 5B",
  "term_label": "endocytic vesicle"
}